{
  "gene": "UniProtKB:P22557",
  "gene_name": "5-aminolevulinate synthase, erythroid-specific, mitochondrial",
  "gene_symbol": "ALAS2",
  "term_id": "GO:0042541",
  "term_label": "hemoglobin biosynthetic process"
}